{
  "gene_symbol": "STIL",
  "gene": "UniProtKB:Q15468",
  "term_id": "GO:0031023",
  "gene_name": "SCL-interrupting locus protein",
  "term_label": "microtubule organizing center organization"
}